root hair [GO:0035618] (cellular component) Definition: A long, thin projection from a root epidermal cell that contains F-actin and tubulin, and a cell wall. Relationships: is a type of GO:0120025 Note: This term is a child of 'cell projection' and not 'cell hair' to distinguish it from animal cell hairs, which are morphologically distinct. References: PMID:24982600 Sources: PO:0000256